positive regulation of translation in response to endoplasmic reticulum stress [GO:0036493] (biological process) Definition: Any process that activates, or increases the frequency, rate or extent of translation as a result of endoplasmic reticulum stress. Relationships: is a type of GO:0032056; is a type of regulation of translation in response to endoplasmic reticulum stress [GO:0036490] Subtypes: positive regulation of translation initiation in response to endoplasmic reticulum stress [GO:0036494] Sources: GOC:PARL, GOC:bf Also known as: positive regulation of translation in response to ER stress